termination of RNA polymerase I transcription [GO:0006363] (biological process) Also known as: RNA polymerase I transcription termination, transcription termination from Pol I promoter, transcription termination from RNA polymerase I promoter, termination of RNA polymerase I transcription from promoter for nuclear large rRNA transcript, RNA polymerase I transcription termination factor activity References: PMID:10684922, PMID:27371117 Sources: GOC:mah, GOC:txnOH Regulation: regulated by GO:2000730; negatively regulated by GO:2000731; positively regulated by GO:2000732 Relationships: is a type of DNA-templated transcription termination [GO:0006353]; is part of GO:0006360 Definition: A transcription termination process that completes the production of a ribosomal RNA transcript. RNAP I termination requires binding of a terminator protein to specific sequences downstream of the transcription unit.